{
  "gene_name": "Psychosine receptor",
  "gene": "UniProtKB:Q8IYL9",
  "term_id": "GO:0005886",
  "term_label": "plasma membrane",
  "gene_symbol": "GPR65"
}